{
  "term_label": "Unknown molecular function",
  "gene_name": "Vesicle-trafficking protein SEC22b",
  "gene_symbol": "SEC22B",
  "gene": "UniProtKB:O75396",
  "term_id": "UNKNOWN:0001"
}